{
  "gene": "UniProtKB:P40925",
  "term_label": "cytosol",
  "gene_name": "Malate dehydrogenase, cytoplasmic",
  "term_id": "GO:0005829",
  "gene_symbol": "MDH1"
}